{
  "gene": "UniProtKB:O43827",
  "term_id": "GO:0005615",
  "gene_symbol": "ANGPTL7",
  "gene_name": "Angiopoietin-related protein 7",
  "term_label": "extracellular space"
}